{
  "gene_name": "Potassium voltage-gated channel subfamily D member 1",
  "term_label": "potassium ion transmembrane transport",
  "gene_symbol": "KCND1",
  "term_id": "GO:0071805",
  "gene": "UniProtKB:Q9NSA2"
}